{
  "gene": "UniProtKB:A8MUK1",
  "term_label": "cysteine-type deubiquitinase activity",
  "term_id": "GO:0004843",
  "gene_symbol": "USP17L5",
  "gene_name": "Ubiquitin carboxyl-terminal hydrolase 17-like protein 5"
}